{
  "gene_symbol": "OGDH",
  "term_id": "GO:0005739",
  "gene": "UniProtKB:Q02218",
  "term_label": "mitochondrion",
  "gene_name": "2-oxoglutarate dehydrogenase complex component E1"
}